{
  "gene": "UniProtKB:O95786",
  "gene_name": "Antiviral innate immune response receptor RIG-I",
  "term_label": "zinc ion binding",
  "term_id": "GO:0008270",
  "gene_symbol": "RIGI"
}